{
  "gene_name": "Neuroligin-3",
  "gene_symbol": "NLGN3",
  "gene": "UniProtKB:Q9NZ94",
  "term_label": "neurexin family protein binding",
  "term_id": "GO:0042043"
}